meiotic nuclear division [GO:0140013] (biological process) Subtypes: meiosis I [GO:0007127], meiosis II [GO:0007135], male meiotic nuclear division [GO:0007140], female meiotic nuclear division [GO:0007143] Regulation: regulated by regulation of meiotic nuclear division [GO:0040020]; negatively regulated by GO:0045835; positively regulated by GO:0045836 References: PMID:9334324 Relationships: is a type of nuclear division [GO:0000280]; is a type of GO:1903046 Also known as: meiosis Definition: One of the two nuclear divisions that occur as part of the meiotic cell cycle.